{
  "gene_symbol": "HOMER3",
  "term_label": "G protein-coupled glutamate receptor signaling pathway",
  "term_id": "GO:0007216",
  "gene_name": "Homer protein homolog 3",
  "gene": "UniProtKB:Q9NSC5"
}